{
  "term_id": "UNKNOWN:0003",
  "gene_name": "T cell receptor alpha variable 4",
  "term_label": "Unknown cellular component",
  "gene": "UniProtKB:A0A0B4J268",
  "gene_symbol": "TRAV4"
}